{
  "term_label": "positive regulation of intrinsic apoptotic signaling pathway",
  "gene_symbol": "BID",
  "gene": "UniProtKB:P55957",
  "gene_name": "BH3-interacting domain death agonist",
  "term_id": "GO:2001244"
}